{
  "term_id": "GO:0005886",
  "gene_symbol": "SLC27A4",
  "gene_name": "Long-chain fatty acid transport protein 4",
  "term_label": "plasma membrane",
  "gene": "UniProtKB:Q6P1M0"
}